negative regulation of transcription by transcription factor catabolism [GO:0010620] (biological process) Relationships: is a type of proteasome-mediated ubiquitin-dependent protein catabolic process [GO:0043161]; is a type of GO:0045892 Definition: Any process that stops, prevents, or reduces the frequency, rate or extent of DNA-dependent transcription using a mechanism that involves the catabolism of a sequence-specific DNA-binding transcription factor by hydrolysis of its peptide bonds, initiated by the covalent attachment of ubiquitin, and mediated by the proteasome. Sources: GOC:bf, GOC:dph, GOC:tb